{
  "gene_symbol": "OTUB1",
  "term_id": "GO:0004843",
  "gene": "UniProtKB:Q96FW1",
  "gene_name": "Ubiquitin thioesterase OTUB1",
  "term_label": "cysteine-type deubiquitinase activity"
}